{
  "gene": "UniProtKB:O15273",
  "term_label": "sarcomerogenesis",
  "term_id": "GO:0048769",
  "gene_symbol": "TCAP",
  "gene_name": "Telethonin"
}